positive regulation of iron ion transmembrane transport [GO:0034761] (biological process) Subtypes: positive regulation of iron export across plasma membrane [GO:1904040], GO:1904440 Relationships: is a type of GO:0034758; is a type of regulation of iron ion transmembrane transport [GO:0034759]; is a type of GO:1904064; positively regulates GO:0034755 Definition: Any process that activates or increases the frequency, rate or extent of the directed movement of iron ions from one side of a membrane to the other by means of some agent such as a transporter or pore. Also known as: positive regulation of iron ion membrane transport, positive regulation of transmembrane iron ion transport, positive regulation of transmembrane iron transport, up regulation of transmembrane iron ion transport, up-regulation of transmembrane iron ion transport, upregulation of transmembrane iron ion transport, activation of transmembrane iron ion transport, stimulation of transmembrane iron ion transport Sources: GOC:mah